{
  "gene_symbol": "SEC13",
  "gene": "UniProtKB:P55735",
  "gene_name": "Protein SEC13 homolog",
  "term_id": "GO:0006606",
  "term_label": "protein import into nucleus"
}